{
  "gene_name": "Leucine-rich repeat-containing protein 36",
  "gene_symbol": "LRRC36",
  "gene": "UniProtKB:Q1X8D7",
  "term_id": "UNKNOWN:0003",
  "term_label": "Unknown cellular component"
}